{
  "term_id": "GO:0003924",
  "term_label": "GTPase activity",
  "gene_symbol": "GNA12",
  "gene": "UniProtKB:Q03113",
  "gene_name": "Guanine nucleotide-binding protein subunit alpha-12"
}